diadenosine polyphosphate metabolic process [GO:0015959] (biological process) Also known as: diadenosine polyphosphate metabolism Relationships: is a type of nucleotide metabolic process [GO:0009117] Definition: The chemical reactions and pathways involving diadenosine polyphosphate, a derivative of the nucleoside adenosine with phosphate groups attached. Sources: GOC:ai Subtypes: diadenosine polyphosphate biosynthetic process [GO:0015960], diadenosine polyphosphate catabolic process [GO:0015961]